{
  "gene_name": "Zinc finger protein 823",
  "term_id": "GO:0006357",
  "gene": "UniProtKB:P16415",
  "gene_symbol": "ZNF823",
  "term_label": "regulation of transcription by RNA polymerase II"
}